{
  "gene_symbol": "NOXA1",
  "gene": "UniProtKB:Q86UR1",
  "term_label": "superoxide anion generation",
  "gene_name": "NADPH oxidase activator 1",
  "term_id": "GO:0042554"
}